{
  "term_id": "GO:1901731",
  "gene_name": "Podoplanin",
  "gene": "UniProtKB:Q86YL7",
  "gene_symbol": "PDPN",
  "term_label": "positive regulation of platelet aggregation"
}